{
  "gene_name": "Cytosolic iron-sulfur assembly component 2B",
  "term_label": "Unknown molecular function",
  "gene": "UniProtKB:Q9Y3D0",
  "gene_symbol": "CIAO2B",
  "term_id": "UNKNOWN:0001"
}